dimethyl sulfoxide reductase complex [GO:0009390] (cellular component) Also known as: dimethyl sulphoxide reductase complex Definition: An enzyme complex that catalyzes the formation of dimethyl sulfide from dimethyl sulfoxide. Relationships: is a type of protein-containing complex [GO:0032991] References: PMID:21357619, PMID:3280546